{
  "gene_name": "Zinc finger protein 322",
  "term_label": "RNA polymerase II cis-regulatory region sequence-specific DNA binding",
  "term_id": "GO:0000978",
  "gene_symbol": "ZNF322",
  "gene": "UniProtKB:Q6U7Q0"
}